vascular endothelial glycocalyx [GO:0120239] (CC) References: PMID:17256154 Sources: GOC:krc Relationships: is a type of glycocalyx [GO:0030112] Also known as: endothelial glycocalyx Definition: The carbohydrate-rich layer lining the vascular endothelium connected to the endothelium through a variety of molecules, mainly proteoglycans and glycoproteins. These form a network in which soluble molecules, either plasma- or endothelium-derived, are incorporated.